{
  "term_id": "GO:0051453",
  "term_label": "regulation of intracellular pH",
  "gene_symbol": "CA2",
  "gene_name": "Carbonic anhydrase 2",
  "gene": "UniProtKB:P00918"
}